{
  "gene": "UniProtKB:A6NJL1",
  "gene_name": "Zinc finger and SCAN domain-containing protein 5B",
  "term_id": "UNKNOWN:0003",
  "gene_symbol": "ZSCAN5B",
  "term_label": "Unknown cellular component"
}